{
  "gene_symbol": "UQCRC2",
  "gene": "UniProtKB:P22695",
  "term_label": "Unknown biological process",
  "term_id": "UNKNOWN:0002",
  "gene_name": "Cytochrome b-c1 complex subunit 2, mitochondrial"
}